{
  "term_id": "GO:0003712",
  "term_label": "transcription coregulator activity",
  "gene_name": "Histone acetyltransferase KAT6A",
  "gene_symbol": "KAT6A",
  "gene": "UniProtKB:Q92794"
}